{
  "term_id": "GO:1905605",
  "gene_name": "Tight junction protein ZO-2",
  "term_label": "positive regulation of blood-brain barrier permeability",
  "gene": "UniProtKB:Q9UDY2",
  "gene_symbol": "TJP2"
}